{
  "gene": "UniProtKB:Q9BYT3",
  "term_id": "GO:0044773",
  "gene_symbol": "STK33",
  "term_label": "mitotic DNA damage checkpoint signaling",
  "gene_name": "Serine_threonine-protein kinase 33"
}